{
  "term_label": "heat shock protein binding",
  "gene": "UniProtKB:P48741",
  "gene_symbol": "HSPA7",
  "term_id": "GO:0031072",
  "gene_name": "Putative heat shock 70 kDa protein 7"
}